glucomannan binding [GO:2001063] (molecular function) Definition: Binding to glucomannan. Sources: GOC:mengo_curators Relationships: is a type of heteropolysaccharide binding [GO:0010297]